regulation of ketone biosynthetic process [GO:0010566] (biological process) Relationships: is a type of regulation of biosynthetic process [GO:0009889]; is a type of GO:0010565; is a type of regulation of small molecule metabolic process [GO:0062012]; regulates ketone biosynthetic process [GO:0042181] Sources: GOC:dph, GOC:tb Definition: Any process that modulates the frequency, rate or extent of the chemical reactions and pathways resulting in the formation of a ketone, carried out by individual cells. Subtypes: regulation of ecdysteroid biosynthetic process [GO:0007554], regulation of ubiquinone biosynthetic process [GO:0010795], regulation of aldosterone biosynthetic process [GO:0032347], regulation of xanthone-containing compound biosynthetic process [GO:1900183], GO:1900379, regulation of kojic acid biosynthetic process [GO:1900394], regulation of emodin biosynthetic process [GO:1900664], GO:1900667, regulation of tensidol A biosynthetic process [GO:1900707], regulation of tensidol B biosynthetic process [GO:1900710], regulation of polyketide biosynthetic process [GO:1900732], GO:1900840, GO:1900843, regulation of naphtho-gamma-pyrone biosynthetic process [GO:1900846], positive regulation of terrequinone A biosynthetic process [GO:1900854], regulation of androst-4-ene-3,17-dione biosynthetic process [GO:1903454], regulation of cortisol biosynthetic process [GO:2000064], GO:2000182, regulation of testosterone biosynthetic process [GO:2000224]